{
  "gene": "UniProtKB:Q9H1C0",
  "gene_name": "Lysophosphatidic acid receptor 5",
  "gene_symbol": "LPAR5",
  "term_label": "Unknown cellular component",
  "term_id": "UNKNOWN:0003"
}